{
  "term_id": "UNKNOWN:0003",
  "gene_name": "Prokineticin-2",
  "gene_symbol": "PROK2",
  "gene": "UniProtKB:Q9HC23",
  "term_label": "Unknown cellular component"
}